{
  "gene_symbol": "HTR5A",
  "term_id": "GO:0007187",
  "term_label": "G protein-coupled receptor signaling pathway, coupled to cyclic nucleotide second messenger",
  "gene": "UniProtKB:P47898",
  "gene_name": "5-hydroxytryptamine receptor 5A"
}